{
  "term_label": "ciliary tip",
  "term_id": "GO:0097542",
  "gene": "UniProtKB:A5D8V7",
  "gene_name": "Outer dynein arm-docking complex subunit 3",
  "gene_symbol": "ODAD3"
}